glycerone-phosphate O-acyltransferase activity [GO:0016287] (molecular function) Sources: EC:2.3.1.42, RHEA:17657 Definition: Catalysis of the reaction: acyl-CoA + glycerone phosphate = 1-acylglycerone 3-phosphate + CoA. Also known as: acyl-CoA:glycerone-phosphate O-acyltransferase activity, dihydroxyacetone phosphate acyltransferase activity Relationships: is a type of GO:0016413